radial spoke head 2 [GO:0120337] (cellular component) Relationships: is a type of radial spoke head [GO:0001535]; is part of GO:0120334 Also known as: radial spokehead 2 Definition: The portion of the radial spoke 2 that is orthogonal to the elongated stalk and which projects towards the central pair of microtubules within the ciliary axoneme. References: PMID:22754630, PMID:348711799 Sources: GOC:krc